{
  "term_id": "GO:0008210",
  "gene_name": "UDP-glucuronosyltransferase 1A3",
  "term_label": "estrogen metabolic process",
  "gene": "UniProtKB:P35503",
  "gene_symbol": "UGT1A3"
}